{
  "gene_name": "Acyl-protein thioesterase 1",
  "gene_symbol": "LYPLA1",
  "term_id": "GO:0005737",
  "gene": "UniProtKB:O75608",
  "term_label": "cytoplasm"
}